{
  "term_id": "GO:0016125",
  "gene": "UniProtKB:Q9HAW7",
  "gene_symbol": "UGT1A7",
  "term_label": "sterol metabolic process",
  "gene_name": "UDP-glucuronosyltransferase 1A7"
}